{
  "gene_name": "CEP295 N-terminal-like protein",
  "term_id": "GO:0046599",
  "gene_symbol": "CEP295NL",
  "term_label": "regulation of centriole replication",
  "gene": "UniProtKB:Q96MC4"
}